{
  "term_id": "UNKNOWN:0001",
  "term_label": "Unknown molecular function",
  "gene": "UniProtKB:Q9UKA1",
  "gene_name": "F-box_LRR-repeat protein 5",
  "gene_symbol": "FBXL5"
}